{
  "term_id": "GO:0005886",
  "gene_name": "Ephrin type-A receptor 6",
  "gene_symbol": "EPHA6",
  "gene": "UniProtKB:Q9UF33",
  "term_label": "plasma membrane"
}